{
  "gene_symbol": "P2RX5",
  "gene_name": "P2X purinoceptor 5",
  "term_label": "plasma membrane",
  "term_id": "GO:0005886",
  "gene": "UniProtKB:Q93086"
}